negative regulation of transforming growth factor beta receptor signaling pathway [GO:0030512] (biological process) Also known as: down regulation of transforming growth factor beta receptor signaling pathway, down-regulation of transforming growth factor beta receptor signaling pathway, downregulation of transforming growth factor beta receptor signaling pathway, negative regulation of TGF-beta receptor signaling pathway, negative regulation of TGFbeta receptor signaling pathway, negative regulation of transforming growth factor beta receptor signalling pathway, inhibition of transforming growth factor beta receptor signaling pathway Relationships: is a type of regulation of transforming growth factor beta receptor signaling pathway [GO:0017015]; is a type of GO:0090101; negatively regulates transforming growth factor beta receptor signaling pathway [GO:0007179] Sources: GOC:mah Subtypes: sequestering of TGFbeta in extracellular matrix [GO:0035583] Definition: Any process that stops, prevents, or reduces the frequency, rate or extent of any TGF-beta receptor signaling pathway.